{
  "term_id": "GO:0005819",
  "gene": "UniProtKB:O00139",
  "term_label": "spindle",
  "gene_name": "Kinesin-like protein KIF2A",
  "gene_symbol": "KIF2A"
}